{
  "term_id": "GO:0016176",
  "term_label": "superoxide-generating NADPH oxidase activator activity",
  "gene": "UniProtKB:Q8NFA2",
  "gene_symbol": "NOXO1",
  "gene_name": "NADPH oxidase organizer 1"
}